{
  "gene_symbol": "DTL",
  "gene": "UniProtKB:Q9NZJ0",
  "term_id": "GO:0043161",
  "term_label": "proteasome-mediated ubiquitin-dependent protein catabolic process",
  "gene_name": "Denticleless protein homolog"
}